glucuronate transmembrane transporter activity [GO:0015135] (molecular function) Definition: Enables the transfer of glucuronate from one side of a membrane to the other. Glucuronate is the uronic acid formally derived from glucose by oxidation of the hydroxymethylene group at C-6 to a carboxyl group. Relationships: is a type of GO:0046943; is part of glucuronate transmembrane transport [GO:0015738] Sources: GOC:ai Subtypes: D-glucuronate transmembrane transporter activity [GO:0042880]